{
  "term_id": "GO:0000122",
  "term_label": "negative regulation of transcription by RNA polymerase II",
  "gene_name": "Melanoma-associated antigen C3",
  "gene": "UniProtKB:Q8TD91",
  "gene_symbol": "MAGEC3"
}